{
  "term_label": "Unknown molecular function",
  "gene_name": "Large ribosomal subunit protein mL53",
  "gene_symbol": "MRPL53",
  "gene": "UniProtKB:Q96EL3",
  "term_id": "UNKNOWN:0001"
}